{
  "gene": "UniProtKB:Q96MC9",
  "term_id": "UNKNOWN:0002",
  "gene_name": "Putative uncharacterized protein IKBKE-AS1",
  "gene_symbol": "IKBKE-AS1",
  "term_label": "Unknown biological process"
}